{
  "gene_symbol": "MUC6",
  "gene_name": "Mucin-6",
  "gene": "UniProtKB:Q6W4X9",
  "term_id": "GO:0005201",
  "term_label": "extracellular matrix structural constituent"
}